{
  "term_label": "ubiquitin protein ligase activity",
  "gene_symbol": "SHPRH",
  "gene": "UniProtKB:Q149N8",
  "term_id": "GO:0061630",
  "gene_name": "E3 ubiquitin-protein ligase SHPRH"
}